{
  "gene_name": "Chymotrypsin-like elastase family member 1",
  "term_id": "GO:0005615",
  "gene": "UniProtKB:Q9UNI1",
  "gene_symbol": "CELA1",
  "term_label": "extracellular space"
}